{
  "term_label": "ATP binding",
  "gene_name": "Regulator of telomere elongation helicase 1",
  "term_id": "GO:0005524",
  "gene_symbol": "RTEL1",
  "gene": "UniProtKB:Q9NZ71"
}